{
  "term_id": "UNKNOWN:0001",
  "gene_name": "Phorbol-12-myristate-13-acetate-induced protein 1",
  "gene_symbol": "PMAIP1",
  "gene": "UniProtKB:Q13794",
  "term_label": "Unknown molecular function"
}